{
  "gene_name": "Chromodomain-helicase-DNA-binding protein 9",
  "gene": "UniProtKB:Q3L8U1",
  "term_id": "UNKNOWN:0001",
  "gene_symbol": "CHD9",
  "term_label": "Unknown molecular function"
}